{
  "gene_name": "Interleukin-6",
  "gene_symbol": "IL6",
  "term_id": "GO:0006954",
  "term_label": "inflammatory response",
  "gene": "UniProtKB:P05231"
}